{
  "term_label": "mitochondrial matrix",
  "gene_name": "Transcription termination factor 2, mitochondrial",
  "term_id": "GO:0005759",
  "gene": "UniProtKB:Q49AM1",
  "gene_symbol": "MTERF2"
}